{
  "term_id": "GO:0008273",
  "gene_symbol": "SLC24A4",
  "gene_name": "Sodium_potassium_calcium exchanger 4",
  "term_label": "calcium, potassium:sodium antiporter activity",
  "gene": "UniProtKB:Q8NFF2"
}